{
  "term_id": "GO:0006099",
  "term_label": "tricarboxylic acid cycle",
  "gene_symbol": "IDH1",
  "gene": "UniProtKB:O75874",
  "gene_name": "Isocitrate dehydrogenase [NADP] cytoplasmic"
}